positive regulation of chromatin organization [GO:1905269] (biological process) Definition: Any process that activates or increases the frequency, rate or extent of chromatin organization. Relationships: is a type of regulation of chromatin organization [GO:1902275]; is a type of positive regulation of chromosome organization [GO:2001252]; positively regulates chromatin organization [GO:0006325] Also known as: positive regulation of chromatin organisation, positive regulation of establishment or maintenance of chromatin architecture, up regulation of chromatin organisation, up regulation of chromatin organization, up regulation of establishment or maintenance of chromatin architecture, up-regulation of chromatin organisation, up-regulation of chromatin organization, up-regulation of establishment or maintenance of chromatin architecture, upregulation of chromatin assembly or disassembly, upregulation of chromatin organisation, upregulation of chromatin organization, upregulation of establishment or maintenance of chromatin architecture, activation of chromatin assembly or disassembly, activation of chromatin organisation, activation of chromatin organization, activation of establishment or maintenance of chromatin architecture, stimulation of chromatin assembly or disassembly, positive regulation of chromatin assembly or disassembly, positive regulation of chromatin assembly/disassembly, positive regulation of chromatin modification, up regulation of chromatin assembly or disassembly, up-regulation of chromatin assembly or disassembly References: PMID:654321 Sources: GOC:TermGenie, GOC:pr, GOC:vw, GO_REF:0000058 Subtypes: GO:0031453, GO:0120263, positive regulation of nucleosome disassembly [GO:0140887]